{
  "gene_symbol": "UNC93A",
  "term_id": "UNKNOWN:0001",
  "gene": "UniProtKB:Q86WB7",
  "term_label": "Unknown molecular function",
  "gene_name": "Protein unc-93 homolog A"
}